{
  "gene_symbol": "QDPR",
  "gene": "UniProtKB:P09417",
  "term_label": "NADH binding",
  "gene_name": "Dihydropteridine reductase",
  "term_id": "GO:0070404"
}